{
  "gene": "UniProtKB:Q8N4C7",
  "term_label": "endomembrane system",
  "term_id": "GO:0012505",
  "gene_name": "Syntaxin-19",
  "gene_symbol": "STX19"
}